{
  "gene_symbol": "NIM1K",
  "term_id": "GO:0035556",
  "gene": "UniProtKB:Q8IY84",
  "term_label": "intracellular signal transduction",
  "gene_name": "Serine_threonine-protein kinase NIM1"
}